dephospho-CoA kinase activity [GO:0004140] (MF) Sources: EC:2.7.1.24, RHEA:18245 Definition: Catalysis of the reaction: 3'-dephospho-CoA + ATP = ADP + CoA + 2 H+. Relationships: is a type of kinase activity [GO:0016301]; is a type of phosphotransferase activity, alcohol group as acceptor [GO:0016773] Also known as: 3'-dephospho-CoA kinase activity, ATP:dephospho-CoA 3'-phosphotransferase activity, dephosphocoenzyme A kinase (phosphorylating), dephosphocoenzyme A kinase activity